fatty acid 2-hydroxylase activity [GO:0080132] (molecular function) Relationships: is a type of GO:0016716 Subtypes: GO:0102771, free fatty acid 2-hydroxylase activity [GO:0120520], GO:0120521 Definition: Catalysis of the hydroxylation of the C-2 position in a fatty acid. The 2-hydroxylation may occur on free fatty acids or within the fatty acyl chain of a sphingolipid. References: PMID:36902339 Also known as: fatty acid alpha-hydroxylase activity